{
  "gene_symbol": "SDC2",
  "term_label": "dendrite morphogenesis",
  "term_id": "GO:0048813",
  "gene": "UniProtKB:P34741",
  "gene_name": "Syndecan-2"
}